{
  "gene": "UniProtKB:Q53FA7",
  "term_id": "GO:0003960",
  "gene_symbol": "TP53I3",
  "gene_name": "Quinone oxidoreductase PIG3",
  "term_label": "quinone reductase (NADPH) activity"
}